regulation of chondrocyte differentiation involved in endochondral bone morphogenesis [GO:1902738] (biological process) Definition: Any process that modulates the rate, frequency, or extent of the process in which a chondroblast acquires specialized structural and/or functional features of a chondrocyte that will contribute to the development of a bone. A chondrocyte is a polymorphic cell that forms cartilage. Relationships: is a type of regulation of chondrocyte differentiation [GO:0032330]; is a type of GO:1903010; is a type of regulation of animal organ morphogenesis [GO:2000027]; regulates GO:0003413 References: PMID:8662546 Sources: GOC:TermGenie, GO_REF:0000058 Subtypes: GO:1902733